{
  "gene": "UniProtKB:A0A087WT01",
  "term_id": "UNKNOWN:0001",
  "gene_name": "T cell receptor alpha variable 27",
  "term_label": "Unknown molecular function",
  "gene_symbol": "TRAV27"
}